negative regulation of peroxisome proliferator activated receptor signaling pathway [GO:0035359] (biological process) Also known as: negative regulation of PPAR signaling pathway, negative regulation of peroxisome proliferator activated receptor signalling pathway, negative regulation of peroxisome proliferator-activated receptor signaling pathway Definition: Any process that stops, prevents, or reduces the frequency, rate or extent of the peroxisome proliferator activated receptor signaling pathway. Relationships: is a type of regulation of peroxisome proliferator activated receptor signaling pathway [GO:0035358]; is a type of GO:1902532; negatively regulates peroxisome proliferator activated receptor signaling pathway [GO:0035357] Sources: GOC:bf